{
  "term_label": "translational termination",
  "gene": "UniProtKB:Q9Y5R4",
  "gene_name": "MTRF1L release factor glutamine methyltransferase",
  "gene_symbol": "HEMK1",
  "term_id": "GO:0006415"
}